{
  "term_label": "DNA-binding transcription factor activity, RNA polymerase II-specific",
  "term_id": "GO:0000981",
  "gene": "UniProtKB:Q8NHV9",
  "gene_name": "Rhox homeobox family member 1",
  "gene_symbol": "RHOXF1"
}